{
  "gene": "UniProtKB:Q8IUB5",
  "term_label": "serine-type endopeptidase inhibitor activity",
  "term_id": "GO:0004867",
  "gene_name": "WAP four-disulfide core domain protein 13",
  "gene_symbol": "WFDC13"
}